{
  "gene_name": "Zinc finger protein 611",
  "gene_symbol": "ZNF611",
  "term_label": "nucleus",
  "term_id": "GO:0005634",
  "gene": "UniProtKB:Q8N823"
}